{
  "gene": "UniProtKB:Q9P2R6",
  "gene_name": "Arginine-glutamic acid dipeptide repeats protein",
  "term_label": "Unknown biological process",
  "term_id": "UNKNOWN:0002",
  "gene_symbol": "RERE"
}